O-fucosylpeptide 3-beta-N-acetylglucosaminyltransferase activity [GO:0033829] (MF) Also known as: O-fucosylpeptide beta-1,3-N-acetylglucosaminyltransferase activity, UDP-D-GlcNAc:O-L-fucosylpeptide 3-beta-N-acetyl-D-glucosaminyltransferase activity Definition: Catalysis of the transfer of a beta-D-GlcNAc residue from UDP-D-GlcNAc to the fucose residue of a fucosylated protein acceptor. Sources: EC:2.4.1.222 Relationships: is a type of acetylglucosaminyltransferase activity [GO:0008375]